{
  "gene_symbol": "SFR1",
  "term_label": "positive regulation of DNA-templated transcription",
  "term_id": "GO:0045893",
  "gene_name": "Swi5-dependent recombination DNA repair protein 1 homolog",
  "gene": "UniProtKB:Q86XK3"
}